{
  "gene_symbol": "APOC1",
  "gene": "UniProtKB:P02654",
  "gene_name": "Apolipoprotein C-I",
  "term_label": "negative regulation of very-low-density lipoprotein particle clearance",
  "term_id": "GO:0010916"
}